{
  "gene": "UniProtKB:Q9HB96",
  "term_label": "Unknown molecular function",
  "gene_name": "Fanconi anemia group E protein",
  "gene_symbol": "FANCE",
  "term_id": "UNKNOWN:0001"
}